{
  "gene_symbol": "GCNA",
  "term_label": "Unknown molecular function",
  "term_id": "UNKNOWN:0001",
  "gene_name": "Germ cell nuclear acidic protein",
  "gene": "UniProtKB:Q96QF7"
}